{
  "term_id": "GO:0017015",
  "gene_name": "Neuronal regeneration-related protein",
  "gene": "UniProtKB:Q16612",
  "term_label": "regulation of transforming growth factor beta receptor signaling pathway",
  "gene_symbol": "NREP"
}